{
  "gene": "UniProtKB:Q9H8N7",
  "gene_name": "Zinc finger protein 395",
  "term_label": "DNA-binding transcription factor activity",
  "gene_symbol": "ZNF395",
  "term_id": "GO:0003700"
}